magnetoreception [GO:0050958] (biological process) Relationships: is a type of sensory perception [GO:0007600] Also known as: magnetoception, sensory perception of magnetic field Subtypes: GO:0050977, magnetoreception by sensory perception of electrical stimulus [GO:0050978], GO:0050979 References: PMID:15886990 Sources: GOC:ai, Wikipedia:Magnetoception Definition: The series of events required for an organism to receive a stimulus relating to a magnetic field, convert it to a molecular signal, and recognize and characterize the signal. Stimuli may be chemical, mechanical or electrical and interpreting these stimuli allows an organism to determine the orientation of a magnetic field. Magnetoreception also involves the perception of light; birds cannot orient without the presence of short wavelength (blue/green) light.